regulation of Ras protein signal transduction [GO:0046578] (BP) Relationships: is a type of regulation of small GTPase mediated signal transduction [GO:0051056]; regulates Ras protein signal transduction [GO:0007265] Definition: Any process that modulates the frequency, rate or extent of Ras protein signal transduction. Sources: GOC:bf Subtypes: GO:0046579, negative regulation of Ras protein signal transduction [GO:0046580]